{
  "gene_name": "Uncharacterized protein KIAA0825",
  "gene_symbol": "KIAA0825",
  "term_id": "UNKNOWN:0001",
  "gene": "UniProtKB:Q8IV33",
  "term_label": "Unknown molecular function"
}